{
  "term_id": "GO:0031507",
  "term_label": "heterochromatin formation",
  "gene": "UniProtKB:Q8IUE6",
  "gene_symbol": "H2AC21",
  "gene_name": "Histone H2A type 2-B"
}